{
  "term_label": "Unknown molecular function",
  "gene_symbol": "GUSBP11",
  "gene": "UniProtKB:Q6P575",
  "gene_name": "Putative inactive beta-glucuronidase protein GUSBP11",
  "term_id": "UNKNOWN:0001"
}